{
  "gene_name": "Olfactory receptor 8H3",
  "gene_symbol": "OR8H3",
  "term_id": "GO:0005549",
  "term_label": "odorant binding",
  "gene": "UniProtKB:Q8N146"
}